6-phosphogluconolactonase activity [GO:0017057] (molecular function) Sources: EC:3.1.1.31, RHEA:12556 Also known as: 6-PGL, 6-phospho-D-glucono-1,5-lactone lactonohydrolase activity, phosphogluconolactonase activity Relationships: is a type of GO:0052689 Definition: Catalysis of the reaction: 6-O-phosphono-D-glucono-1,5-lactone + H2O = 6-phospho-D-gluconate + H+.